{
  "gene": "UniProtKB:Q99615",
  "gene_symbol": "DNAJC7",
  "term_id": "UNKNOWN:0001",
  "term_label": "Unknown molecular function",
  "gene_name": "DnaJ homolog subfamily C member 7"
}